{
  "gene_symbol": "UBE2T",
  "term_id": "GO:0005634",
  "gene_name": "Ubiquitin-conjugating enzyme E2 T",
  "gene": "UniProtKB:Q9NPD8",
  "term_label": "nucleus"
}